box C/D RNP complex [GO:0170049] (cellular component) References: PMID:28505386, PMID:30254138 Also known as: SNORD ribonucleoprotein complex, SNORNP Relationships: is a type of sno(s)RNA-containing ribonucleoprotein complex [GO:0005732] Subtypes: GO:0031428, GO:0170050, GO:0170051, GO:0170052 Definition: A ribonucleoprotein complex consisting of a box C/D type snRNA and three (Archaea) or four (Eukaryotes) core proteins that have diverse functions, including site-specific methylation of rRNA and processing rRNA.